{
  "term_label": "antibody-dependent cellular cytotoxicity",
  "gene_symbol": "FCGR1BP",
  "gene_name": "Putative high affinity immunoglobulin gamma Fc receptor IB",
  "term_id": "GO:0001788",
  "gene": "UniProtKB:Q92637"
}